protein localization to microtubule organizing center [GO:1905508] (biological process) Subtypes: protein localization to centrosome [GO:0071539], protein localization to spindle pole body [GO:0071988], protein localization to equatorial microtubule organizing center [GO:1904759], GO:1905509 Also known as: protein localisation in microtubule organizing center, protein localisation to microtubule organizing center, protein localization in microtubule organizing center Definition: A process in which a protein is transported to, or maintained in, a location within a microtubule organizing center. Relationships: is a type of protein localization to microtubule cytoskeleton [GO:0072698] References: PMID:19001497 Sources: GOC:TermGenie, GO_REF:0000087